neuronal signal transduction [GO:0023041] (biological process) Definition: The process in which an activated neuronal cell receptor conveys information down a signaling pathway, resulting in a change in the function or state of a cell. This process may be intracellular or intercellular. Regulation: regulated by regulation of neuronal signal transduction [GO:1902847]; negatively regulated by negative regulation of neuronal signal transduction [GO:1902848]; positively regulated by GO:1902849 Relationships: is a type of signal transduction [GO:0007165] Sources: GOC:mtg_signal